cytoplasmic vesicle lumen [GO:0060205] (cellular component) Relationships: is a type of GO:0031983; is a type of intracellular organelle lumen [GO:0070013]; is part of cytoplasmic vesicle [GO:0031410] Definition: The volume enclosed by a cytoplasmic vesicle. Also known as: cytoplasmic membrane-bounded vesicle lumen, cytoplasmic membrane-enclosed vesicle lumen Subtypes: plasma membrane-derived thylakoid lumen [GO:0031979], GO:0034422, esterosome lumen [GO:0034467], melanosome lumen [GO:0034493], synaptic vesicle lumen [GO:0034592], secretory granule lumen [GO:0034774], clathrin-sculpted acetylcholine transport vesicle lumen [GO:0060202], clathrin-sculpted glutamate transport vesicle lumen [GO:0060204], clathrin-sculpted gamma-aminobutyric acid transport vesicle lumen [GO:0061201], clathrin-sculpted monoamine transport vesicle lumen [GO:0070082], Golgi-associated vesicle lumen [GO:0070931], GO:0098566, spine apparatus lumen [GO:0098899], COPI-coated vesicle lumen [GO:0106172], COPII-coated vesicle lumen [GO:0106173], phagolysosome vesicle lumen [GO:0106174], cytolytic granule lumen [GO:1904856] Sources: GOC:dph, GOC:vesicles